{
  "gene_name": "Arginase-1",
  "term_label": "cytoplasm",
  "gene": "UniProtKB:P05089",
  "gene_symbol": "ARG1",
  "term_id": "GO:0005737"
}